positive regulation of striated muscle contraction [GO:0045989] (biological process) Sources: GOC:go_curators Relationships: is a type of regulation of striated muscle contraction [GO:0006942]; is a type of GO:0045933; positively regulates striated muscle contraction [GO:0006941] Definition: Any process that activates or increases the frequency, rate or extent of striated muscle contraction. Subtypes: positive regulation of tonic skeletal muscle contraction [GO:0014747], positive regulation of skeletal muscle contraction by regulation of release of sequestered calcium ion [GO:0014810], positive regulation of fast-twitch skeletal muscle fiber contraction [GO:0031448], GO:0031451, positive regulation of cardiac muscle contraction [GO:0060452] Also known as: up regulation of striated muscle contraction, up-regulation of striated muscle contraction, upregulation of striated muscle contraction, activation of striated muscle contraction, stimulation of striated muscle contraction